{
  "term_id": "GO:0042742",
  "gene_symbol": "DEFB130A",
  "gene": "UniProtKB:P0DP74",
  "term_label": "defense response to bacterium",
  "gene_name": "Beta-defensin 130A"
}